{
  "gene_symbol": "BABAM2",
  "gene_name": "BRISC and BRCA1-A complex member 2",
  "term_label": "Unknown molecular function",
  "gene": "UniProtKB:Q9NXR7",
  "term_id": "UNKNOWN:0001"
}